{
  "gene": "UniProtKB:Q9BQ39",
  "term_id": "GO:0005730",
  "gene_symbol": "DDX50",
  "term_label": "nucleolus",
  "gene_name": "ATP-dependent RNA helicase DDX50"
}